{
  "term_id": "GO:0005634",
  "gene": "UniProtKB:Q9P2J8",
  "gene_symbol": "ZNF624",
  "term_label": "nucleus",
  "gene_name": "Zinc finger protein 624"
}